{
  "gene": "UniProtKB:Q6ZTR7",
  "term_label": "ciliary basal body",
  "gene_symbol": "CIBAR2",
  "term_id": "GO:0036064",
  "gene_name": "CBY1-interacting BAR domain-containing protein 2"
}